{
  "gene": "UniProtKB:Q16873",
  "gene_symbol": "LTC4S",
  "gene_name": "Leukotriene C4 synthase",
  "term_id": "GO:0005635",
  "term_label": "nuclear envelope"
}